{
  "term_label": "prefoldin complex",
  "term_id": "GO:0016272",
  "gene": "UniProtKB:Q9NQP4",
  "gene_name": "Prefoldin subunit 4",
  "gene_symbol": "PFDN4"
}